negative regulation of microtubule polymerization or depolymerization [GO:0031111] (biological process) Definition: Any process that stops, prevents, or reduces the frequency, rate or extent of microtubule polymerization or depolymerization. Sources: GOC:mah Subtypes: negative regulation of microtubule depolymerization [GO:0007026], negative regulation of microtubule polymerization [GO:0031115] Also known as: down regulation of microtubule polymerization or depolymerization, down-regulation of microtubule polymerization or depolymerization, downregulation of microtubule polymerization or depolymerization, inhibition of microtubule polymerization or depolymerization Relationships: is a type of regulation of microtubule polymerization or depolymerization [GO:0031110]; is a type of negative regulation of cytoskeleton organization [GO:0051494]; negatively regulates GO:0031109